positive regulation of epiboly involved in gastrulation with mouth forming second [GO:1904088] (biological process) Also known as: up regulation of epiboly involved in gastrulation with mouth forming second, up-regulation of epiboly involved in gastrulation with mouth forming second, upregulation of epiboly involved in gastrulation with mouth forming second, activation of epiboly involved in gastrulation with mouth forming second Definition: Any process that activates or increases the frequency, rate or extent of epiboly involved in gastrulation with mouth forming second. References: PMID:24892953 Sources: GOC:TermGenie, GO_REF:0000058 Relationships: is a type of regulation of epiboly involved in gastrulation with mouth forming second [GO:1904086]; is a type of positive regulation of morphogenesis of an epithelium [GO:1905332]; positively regulates epiboly involved in gastrulation with mouth forming second [GO:0055113]